{
  "gene_symbol": "UBE2E3",
  "gene_name": "Ubiquitin-conjugating enzyme E2 E3",
  "term_label": "protein K48-linked ubiquitination",
  "term_id": "GO:0070936",
  "gene": "UniProtKB:Q969T4"
}